{
  "term_label": "positive regulation of immunoglobulin production",
  "gene": "UniProtKB:P78552",
  "term_id": "GO:0002639",
  "gene_name": "Interleukin-13 receptor subunit alpha-1",
  "gene_symbol": "IL13RA1"
}